{
  "term_label": "G1/S transition of mitotic cell cycle",
  "term_id": "GO:0000082",
  "gene_name": "G1_S-specific cyclin-D1",
  "gene_symbol": "CCND1",
  "gene": "UniProtKB:P24385"
}